{
  "gene_symbol": "BATF",
  "term_id": "GO:0006357",
  "term_label": "regulation of transcription by RNA polymerase II",
  "gene": "UniProtKB:Q16520",
  "gene_name": "Basic leucine zipper transcriptional factor ATF-like"
}